{
  "term_label": "microtubule cytoskeleton organization",
  "term_id": "GO:0000226",
  "gene_name": "Tubulin polyglutamylase TTLL7",
  "gene": "UniProtKB:Q6ZT98",
  "gene_symbol": "TTLL7"
}